cADPR-sensitive calcium-release channel activity [GO:0072346] (molecular function) Relationships: is a type of intracellularly gated calcium channel activity [GO:0015278] References: PMID:11752598 Definition: Enables the transmembrane transfer of a calcium ion by a channel that opens when cyclic adenosine diphosphate ribose (cADPR) has been bound by the channel complex or one of its constituent parts.